specification of petal identity [GO:0010095] (BP) Definition: The process in which a floral organ primordium acquires petal identity. Identity is considered to be the aggregate of characteristics by which a structure is recognized. Sources: GOC:tair_curators Relationships: is a type of specification of floral organ identity [GO:0010093]; is part of petal formation [GO:0048451]